{
  "gene_symbol": "LRR1",
  "term_label": "Unknown molecular function",
  "term_id": "UNKNOWN:0001",
  "gene_name": "Leucine-rich repeat protein 1",
  "gene": "UniProtKB:Q96L50"
}